{
  "term_label": "transcription factor TFIIH core complex",
  "term_id": "GO:0000439",
  "gene_symbol": "GTF2H3",
  "gene": "UniProtKB:Q13889",
  "gene_name": "General transcription factor IIH subunit 3"
}